channel activator activity [GO:0099103] (molecular function) Subtypes: GO:0099104 Also known as: channel gating activity Relationships: is a type of channel regulator activity [GO:0016247]; is a type of transporter activator activity [GO:0141109]; positively regulates channel activity [GO:0015267] Sources: GOC:dos Definition: Direct interaction with a channel (binding or modification), resulting in its opening. A channel catalyzes energy-independent facilitated diffusion, mediated by passage of a solute through a transmembrane aqueous pore or channel.